{
  "term_id": "GO:0005634",
  "gene_symbol": "NEDD8",
  "term_label": "nucleus",
  "gene": "UniProtKB:Q15843",
  "gene_name": "NEDD8"
}